{
  "gene_symbol": "ZBTB17",
  "term_label": "negative regulation of transcription by RNA polymerase II",
  "gene": "UniProtKB:Q13105",
  "term_id": "GO:0000122",
  "gene_name": "Zinc finger and BTB domain-containing protein 17"
}